{
  "term_label": "Unknown cellular component",
  "gene": "UniProtKB:Q59EK9",
  "term_id": "UNKNOWN:0003",
  "gene_name": "RUN domain-containing protein 3A",
  "gene_symbol": "RUNDC3A"
}